glycolipid binding [GO:0051861] (molecular function) Subtypes: GO:0034235, GO:0043208, sulfatide binding [GO:0120146] Relationships: is a type of lipid binding [GO:0008289]; is a type of carbohydrate derivative binding [GO:0097367] Definition: Binding to a glycolipid, any compound containing one or more monosaccharide residues bound by a glycosidic linkage to a hydrophobic group such as an acylglycerol, a sphingoid, a ceramide (N-acylsphingoid) or a prenyl phosphate. References: PMID:19635802